{
  "gene": "UniProtKB:P51809",
  "gene_symbol": "VAMP7",
  "term_id": "GO:0006906",
  "gene_name": "Vesicle-associated membrane protein 7",
  "term_label": "vesicle fusion"
}